neuron to neuron synapse [GO:0098984] (cellular component) Sources: GOC:dos Relationships: is a type of synapse [GO:0045202] Subtypes: asymmetric synapse [GO:0032279], symmetric synapse [GO:0032280], GO:0098686 Definition: A synapse in which pre and post-synaptic cells are neurons.